regulation of nucleobase-containing compound transport [GO:0032239] (biological process) Subtypes: GO:0032240, GO:0032241, GO:0032242, GO:0035345, regulation of thymine transport [GO:0035365], regulation of RNA import into nucleus [GO:0046828], GO:0046831 Also known as: regulation of nucleobase, nucleoside, nucleotide and nucleic acid transport Relationships: is a type of regulation of transport [GO:0051049]; regulates nucleobase-containing compound transport [GO:0015931] Sources: GOC:mah Definition: Any process that modulates the frequency, rate or extent of the directed movement of nucleobases, nucleosides, nucleotides and nucleic acids, into, out of or within a cell, or between cells, by means of some agent such as a transporter or pore.